{
  "gene": "UniProtKB:Q8NHU3",
  "gene_name": "Phosphatidylcholine:ceramide cholinephosphotransferase 2",
  "term_id": "GO:0046513",
  "gene_symbol": "SGMS2",
  "term_label": "ceramide biosynthetic process"
}